{
  "gene_name": "Translocon-associated protein subunit alpha",
  "gene": "UniProtKB:P43307",
  "term_label": "Unknown molecular function",
  "gene_symbol": "SSR1",
  "term_id": "UNKNOWN:0001"
}